{
  "term_label": "DNA damage response",
  "gene": "UniProtKB:Q9BYP7",
  "term_id": "GO:0006974",
  "gene_name": "Serine_threonine-protein kinase WNK3",
  "gene_symbol": "WNK3"
}